{
  "gene_name": "NMDA receptor synaptonuclear signaling and neuronal migration factor",
  "gene_symbol": "NSMF",
  "term_label": "Unknown molecular function",
  "gene": "UniProtKB:Q6X4W1",
  "term_id": "UNKNOWN:0001"
}